mitotic cell cycle checkpoint signaling [GO:0007093] (biological process) Relationships: is a type of cell cycle checkpoint signaling [GO:0000075]; is a type of GO:0045930; is a type of GO:1903047 Definition: A signaling process that ensures accurate chromosome replication and segregation by preventing progression through a mitotic cell cycle until conditions are suitable for the cell to proceed to the next stage. Also known as: mitotic cell cycle checkpoint, signal transduction involved in mitotic cell cycle checkpoint, signal transduction involved in mitotic G2/M transition checkpoint, signal transduction involved in mitotic cell cycle G1/S checkpoint, mitotic checkpoint Subtypes: mitotic cell size control checkpoint signaling [GO:0031567], mitotic DNA integrity checkpoint signaling [GO:0044774], mitotic G2/M transition checkpoint [GO:0044818], mitotic G1/S transition checkpoint signaling [GO:0044819], mitotic cytokinesis checkpoint signaling [GO:0044878], mitotic morphogenesis checkpoint signaling [GO:0044879], mitotic spindle checkpoint signaling [GO:0071174], signal transduction involved in cytokinesis checkpoint [GO:0072398] Sources: GOC:mtg_cell_cycle